{
  "gene_name": "Protein MEMO1",
  "gene_symbol": "MEMO1",
  "term_id": "UNKNOWN:0001",
  "gene": "UniProtKB:Q9Y316",
  "term_label": "Unknown molecular function"
}